D-lactate biosynthetic process from methylglyoxal via (R)-lactaldehyde [GO:0019248] (biological process) Also known as: D-lactate anabolism from methylglyoxal via (R)-lactaldehyde, D-lactate formation from methylglyoxal via (R)-lactaldehyde, D-lactate synthesis from methylglyoxal via (R)-lactaldehyde Definition: The chemical reactions and pathways resulting in the formation of D-lactate from methylglyoxal, via the intermediate (R)-lactaldehyde. Relationships: is a type of lactate biosynthetic process [GO:0019249]; is a type of methylglyoxal catabolic process to lactate [GO:0061727]; has part oxidoreductase activity, acting on the aldehyde or oxo group of donors, NAD or NADP as acceptor [GO:0016620]; has part methylglyoxal reductase (NADH) activity [GO:0019170] Sources: GOC:dph, GOC:go_curators, MetaCyc:MGLDLCTANA-PWY